{
  "gene_name": "Regulating synaptic membrane exocytosis protein 4",
  "term_label": "Unknown biological process",
  "gene_symbol": "RIMS4",
  "gene": "UniProtKB:Q9H426",
  "term_id": "UNKNOWN:0002"
}